lipopolysaccharide receptor complex [GO:0046696] (CC) Note: Note that this term should not be used to refer to CD14 alone, but the multiprotein receptor complex that it is part of. Relationships: is a type of receptor complex [GO:0043235]; is a type of GO:0098796 References: PMID:11706042, PMID:9665271 Also known as: LPS receptor complex Definition: A multiprotein complex that consists of at least three proteins, CD14, TLR4, and MD-2, each of which is glycosylated and which functions as a lipopolysaccharide (LPS) receptor that primes the innate immune response against bacterial pathogens.